BRCA2-MAGE-D1 complex [GO:0033593] (cellular component) Definition: A heterodimeric protein complex formed of BRCA2 and MAGE-D1; may mediate the synergistic activities of the two proteins in regulating cell growth. Relationships: is a type of intracellular protein-containing complex [GO:0140535] References: PMID:15930293